mitotic spindle microtubule depolymerization [GO:1990755] (biological process) Relationships: is a type of GO:0007019 Definition: The removal of tubulin heterodimers from one or both ends of a microtubule that is part of the mitotic spindle. Also known as: mitotic spindle microtubule depolymerisation References: PMID:25253718